NAD+-protein-aspartate ADP-ribosyltransferase activity [GO:0140806] (molecular function) Relationships: is_a NAD+-protein mono-ADP-ribosyltransferase activity [GO:1990404] References: PMID:19764761, PMID:25043379 Sources: RHEA:54424 Definition: Catalysis of the reaction: L-aspartyl-[protein] + NAD+ = 4-O-(ADP-D-ribosyl)-L-aspartyl-[protein] + nicotinamide.